{
  "term_id": "UNKNOWN:0001",
  "gene_name": "Cartilage acidic protein 1",
  "gene": "UniProtKB:Q9NQ79",
  "term_label": "Unknown molecular function",
  "gene_symbol": "CRTAC1"
}